{
  "term_id": "GO:0019901",
  "gene": "UniProtKB:Q9H568",
  "term_label": "protein kinase binding",
  "gene_symbol": "ACTL8",
  "gene_name": "Actin-like protein 8"
}